negative regulation of monocyte antigen processing and presentation [GO:0002614] (biological process) Sources: GOC:add Also known as: down regulation of monocyte antigen processing and presentation, down-regulation of monocyte antigen processing and presentation, downregulation of monocyte antigen processing and presentation, inhibition of monocyte antigen processing and presentation Definition: Any process that stops, prevents, or reduces the frequency, rate, or extent of monocyte antigen processing and presentation. Relationships: is a type of GO:0002578; is a type of regulation of monocyte antigen processing and presentation [GO:0002613]; negatively regulates monocyte antigen processing and presentation [GO:0002471]